{
  "term_id": "GO:0005615",
  "gene_symbol": "IFNA6",
  "gene_name": "Interferon alpha-6",
  "term_label": "extracellular space",
  "gene": "UniProtKB:P05013"
}